{
  "term_label": "Unknown cellular component",
  "gene_symbol": "HS6ST2",
  "term_id": "UNKNOWN:0003",
  "gene_name": "Heparan-sulfate 6-O-sulfotransferase 2",
  "gene": "UniProtKB:Q96MM7"
}